{
  "gene_symbol": "MROH2B",
  "term_id": "GO:0005737",
  "term_label": "cytoplasm",
  "gene": "UniProtKB:Q7Z745",
  "gene_name": "Maestro heat-like repeat-containing protein family member 2B"
}